aminopeptidase activity [GO:0004177] (molecular function) Relationships: is_a exopeptidase activity [GO:0008238] References: PMID:24157837 Sources: EC:3.4.11.-, https://www.ebi.ac.uk/merops/about/glossary.shtml#AMINOPEPTIDASE Subtypes: GO:0004230, GO:0004239, alanyl aminopeptidase activity [GO:0016285], tripeptide aminopeptidase activity [GO:0045148], cysteine-type aminopeptidase activity [GO:0070005], GO:0070006, serine-type aminopeptidase activity [GO:0070009] Definition: Catalysis of the hydrolysis of a single N-terminal amino acid residue from a polypeptide chain.